negative regulation of growth hormone secretion [GO:0060125] (biological process) Sources: GOC:dph Definition: Any process that decreases or stops the frequency, rate or extent of the regulated release of growth hormone from a cell. Relationships: is_a regulation of growth hormone secretion [GO:0060123]; is a type of GO:0090278; RO_0002212 GO:0030252